{
  "gene_symbol": "APRT",
  "term_id": "GO:0016208",
  "gene": "UniProtKB:P07741",
  "term_label": "AMP binding",
  "gene_name": "Adenine phosphoribosyltransferase"
}